{
  "term_label": "adherens junction organization",
  "gene_symbol": "CDH19",
  "term_id": "GO:0034332",
  "gene_name": "Cadherin-19",
  "gene": "UniProtKB:Q9H159"
}